{
  "gene_symbol": "SMC1A",
  "gene": "UniProtKB:Q14683",
  "term_label": "DNA binding",
  "gene_name": "Structural maintenance of chromosomes protein 1A",
  "term_id": "GO:0003677"
}